phosphagen catabolic process [GO:0042397] (biological process) Definition: The chemical reactions and pathways resulting in the breakdown of phosphagen, any of a group of guanidine phosphates that occur in muscle and can be used to regenerate ATP from ADP during muscular contraction. Sources: GOC:jl, ISBN:0198506732 Subtypes: phosphoarginine catabolic process [GO:0046313], phosphocreatine catabolic process [GO:0046315] Relationships: is a type of GO:0006796; is a type of GO:0042219; is a type of GO:0046434 Also known as: phosphagen breakdown, phosphagen catabolism, phosphagen degradation